{
  "term_label": "Unknown molecular function",
  "gene_symbol": "PDCD1",
  "gene_name": "Programmed cell death protein 1",
  "gene": "UniProtKB:Q15116",
  "term_id": "UNKNOWN:0001"
}